{
  "term_label": "intracellular manganese ion homeostasis",
  "term_id": "GO:0030026",
  "gene_name": "Natural resistance-associated macrophage protein 1",
  "gene_symbol": "SLC11A1",
  "gene": "UniProtKB:P49279"
}